{
  "gene_name": "Solute carrier family 25 member 16",
  "gene": "UniProtKB:P16260",
  "term_label": "mitochondrial inner membrane",
  "gene_symbol": "SLC25A16",
  "term_id": "GO:0005743"
}